{
  "term_id": "GO:0007229",
  "gene_symbol": "ITGA8",
  "gene": "UniProtKB:P53708",
  "gene_name": "Integrin alpha-8",
  "term_label": "integrin-mediated signaling pathway"
}